CoA-ligase activity [GO:0016405] (molecular function) Subtypes: GO:0003987, GO:0008756, GO:0016207, GO:0018855, GO:0018856, benzoate-CoA ligase activity [GO:0018858], 4-hydroxybenzoate-CoA ligase activity [GO:0018859], GO:0018860, GO:0018861, GO:0030729, citronellyl-CoA ligase activity [GO:0034823], GO:0042410, 3-hydroxypropionyl-CoA synthetase activity [GO:0043955], phenylacetate-CoA ligase activity [GO:0047475], 3-alpha,7-alpha-dihydroxy-5-beta-cholestanate-CoA ligase activity [GO:0047476], 2-furoate-CoA ligase activity [GO:0047541], biotin-CoA ligase activity [GO:0047707], GO:0047747, phytanate-CoA ligase activity [GO:0050197], oxalate-CoA ligase activity [GO:0050203], GO:0050563, carnitine-CoA ligase activity [GO:0051108], GO:0051109, perillic acid-CoA ligase (AMP-forming) activity [GO:0052686], (3R)-3-isopropenyl-6-oxoheptanoate:CoA ligase (ADP-forming) activity [GO:0052687], (3R)-3-isopropenyl-6-oxoheptanoate:CoA ligase (AMP-forming) activity [GO:0052688], pristanate-CoA ligase activity [GO:0070251], malonyl-CoA synthetase activity [GO:0090409], (E)-caffeate-CoA ligase activity [GO:0106286], trans-cinnamate-CoA ligase activity [GO:0106290], fatty acid-CoA ligase activity [GO:0120515] Relationships: is a type of ligase activity, forming carbon-sulfur bonds [GO:0016877] Sources: GOC:ai Definition: Catalysis of the reaction: substrate + ATP + CoASH = AMP + diphosphate + substrate-CoA.